{
  "gene": "UniProtKB:P14867",
  "gene_name": "Gamma-aminobutyric acid receptor subunit alpha-1",
  "gene_symbol": "GABRA1",
  "term_label": "GABA-A receptor complex",
  "term_id": "GO:1902711"
}